{
  "term_id": "GO:0000978",
  "gene_name": "Iroquois-class homeodomain protein IRX-2",
  "term_label": "RNA polymerase II cis-regulatory region sequence-specific DNA binding",
  "gene_symbol": "IRX2",
  "gene": "UniProtKB:Q9BZI1"
}